CGU codon-amino acid adaptor activity [GO:0033429] (molecular function) Also known as: CGT codon-amino acid adaptor activity, arginine tRNA Relationships: is a type of GO:0030533 Note: Note that in the standard genetic code, CGT codes for arginine. Sources: GOC:mah Definition: A triplet codon-amino acid adaptor activity that recognizes a CGU codon.